positive regulation of interleukin-1 production [GO:0032732] (biological process) Relationships: is a type of positive regulation of cytokine production [GO:0001819]; is a type of GO:0032652; positively regulates interleukin-1 production [GO:0032612] Sources: GOC:mah Definition: Any process that activates or increases the frequency, rate, or extent of interleukin-1 production. Subtypes: positive regulation of interleukin-1 alpha production [GO:0032730], positive regulation of interleukin-1 beta production [GO:0032731] Also known as: positive regulation of IL-1 production, up regulation of interleukin-1 production, up-regulation of interleukin-1 production, upregulation of interleukin-1 production, activation of interleukin-1 production, positive regulation of interleukin-1 biosynthetic process, positive regulation of interleukin-1 secretion, stimulation of interleukin-1 production